{
  "gene_name": "RNA-binding motif, single-stranded-interacting protein 3",
  "gene": "UniProtKB:Q6XE24",
  "term_id": "GO:0008143",
  "term_label": "poly(A) binding",
  "gene_symbol": "RBMS3"
}